{
  "gene_name": "Neuronal acetylcholine receptor subunit alpha-3",
  "gene": "UniProtKB:P32297",
  "term_id": "GO:0022848",
  "gene_symbol": "CHRNA3",
  "term_label": "acetylcholine-gated monoatomic cation-selective channel activity"
}